{
  "term_label": "Unknown cellular component",
  "gene": "UniProtKB:Q16557",
  "term_id": "UNKNOWN:0003",
  "gene_name": "Pregnancy-specific beta-1-glycoprotein 3",
  "gene_symbol": "PSG3"
}